genital disc morphogenesis [GO:0007483] (biological process) Also known as: genital disc metamorphosis Relationships: is a type of GO:0007560; is part of genital disc development [GO:0035215] Sources: GOC:bf, ISBN:0879694238 Definition: The process in which the anatomical structures derived from the genital disc are generated and organized. This includes the transformation of a genital imaginal disc from a monolayered epithelium in the larvae of holometabolous insects into the recognizable adult genital structures, the anal plates and the hind gut.